putrescine biosynthetic process from arginine, via ornithine [GO:0033387] (biological process) Definition: The chemical reactions and pathways resulting in the formation of putrescine, 1,4-diaminobutane, from arginine, via decarboxylation of ornithine. Sources: GOC:mah, MetaCyc:PWY-46 Relationships: is a type of GO:0033388 Also known as: putrescine anabolism from ornithine, putrescine biosynthesis from ornithine, putrescine biosynthetic process from ornithine, putrescine formation from ornithine, putrescine synthesis from ornithine